{
  "term_id": "GO:0033038",
  "gene_name": "Taste receptor type 2 member 8",
  "gene": "UniProtKB:Q9NYW2",
  "term_label": "bitter taste receptor activity",
  "gene_symbol": "TAS2R8"
}